{
  "term_id": "GO:0008017",
  "gene_name": "Nuclear distribution protein nudE-like 1",
  "term_label": "microtubule binding",
  "gene": "UniProtKB:Q9GZM8",
  "gene_symbol": "NDEL1"
}